{
  "term_id": "GO:0005737",
  "gene_name": "Dapper homolog 3",
  "gene": "UniProtKB:Q96B18",
  "gene_symbol": "DACT3",
  "term_label": "cytoplasm"
}